{
  "term_id": "GO:0006783",
  "gene": "UniProtKB:A8MWL7",
  "gene_name": "Transmembrane protein 14DP",
  "term_label": "heme biosynthetic process",
  "gene_symbol": "TMEM14DP"
}